{
  "gene_name": "Uroporphyrinogen decarboxylase",
  "gene_symbol": "UROD",
  "term_label": "uroporphyrinogen decarboxylase activity",
  "term_id": "GO:0004853",
  "gene": "UniProtKB:P06132"
}